{
  "gene": "UniProtKB:P49765",
  "term_label": "sprouting angiogenesis",
  "gene_symbol": "VEGFB",
  "term_id": "GO:0002040",
  "gene_name": "Vascular endothelial growth factor B"
}